{
  "gene_symbol": "MYO7B",
  "term_label": "actin filament organization",
  "gene_name": "Unconventional myosin-VIIb",
  "term_id": "GO:0007015",
  "gene": "UniProtKB:Q6PIF6"
}